phosphoprotein binding [GO:0051219] (molecular function) Definition: Binding to a phosphorylated protein. Sources: GOC:ai Subtypes: protein phosphorylated amino acid binding [GO:0045309] Relationships: is a type of GO:0005515 Also known as: phosphorylated protein binding